positive regulation of cholesterol efflux [GO:0010875] (biological process) Relationships: is a type of regulation of cholesterol efflux [GO:0010874]; is a type of positive regulation of cholesterol transport [GO:0032376]; positively regulates cholesterol efflux [GO:0033344] Sources: GOC:BHF, GOC:dph, GOC:tb Definition: Any process that increases the frequency, rate or extent of cholesterol efflux. Cholesterol efflux is the directed movement of cholesterol, cholest-5-en-3-beta-ol, out of a cell or organelle.